myosin filament disassembly [GO:0031035] (biological process) Subtypes: GO:0031037 Sources: GOC:mah Definition: The disassembly of a filament composed of myosin molecules. Relationships: is a type of GO:0031033; is a type of GO:0032984 Also known as: myosin depolymerization